phenylalanine transport [GO:0015823] (biological process) Subtypes: L-phenylalanine import across plasma membrane [GO:0140925] Relationships: is a type of carboxylic acid transport [GO:0046942]; is a type of GO:0071705 Definition: The directed movement of phenylalanine, 2-amino-3-phenylpropanoic acid, into, out of or within a cell, or between cells, by means of some agent such as a transporter or pore. Sources: GOC:ai Also known as: L-phenylalanine transport